hypotaurine monooxygenase activity [GO:0047822] (molecular function) Relationships: is a type of GO:0016709 Definition: Catalysis of the reaction: H+ + hypotaurine + NADPH + O2 = H2O + NADP+ + taurine. Sources: RHEA:69819 Also known as: hypotaurine dehydrogenase activity